{
  "gene_name": "UNC5C-like protein",
  "gene_symbol": "UNC5CL",
  "gene": "UniProtKB:Q8IV45",
  "term_id": "UNKNOWN:0001",
  "term_label": "Unknown molecular function"
}